{
  "term_id": "UNKNOWN:0002",
  "gene_name": "Putative heat shock protein HSP 90-alpha A4",
  "term_label": "Unknown biological process",
  "gene": "UniProtKB:Q58FG1",
  "gene_symbol": "HSP90AA4P"
}